{
  "gene_name": "Tripartite motif-containing protein 44",
  "gene": "UniProtKB:Q96DX7",
  "term_id": "GO:0005737",
  "term_label": "cytoplasm",
  "gene_symbol": "TRIM44"
}